{
  "gene_symbol": "NEURL2",
  "gene_name": "Neuralized-like protein 2",
  "gene": "UniProtKB:Q9BR09",
  "term_label": "Unknown cellular component",
  "term_id": "UNKNOWN:0003"
}